glyoxylate reductase (NADPH) activity [GO:0030267] (molecular function) Also known as: NADPH-glyoxylate reductase activity, glycolate:NADP+ oxidoreductase activity, glyoxylate reductase (NADP+) Relationships: is a type of glyoxylate reductase activity [GO:0106345] Sources: RHEA:10992 Definition: Catalysis of the reaction: glycolate + NADP+ = glyoxylate + NADPH + H+.